{
  "gene_symbol": "NUBP1",
  "gene_name": "Cytosolic Fe-S cluster assembly factor NUBP1",
  "term_id": "GO:0051536",
  "gene": "UniProtKB:P53384",
  "term_label": "iron-sulfur cluster binding"
}